{
  "gene_symbol": "PRAG1",
  "term_id": "UNKNOWN:0003",
  "gene": "UniProtKB:Q86YV5",
  "gene_name": "Inactive tyrosine-protein kinase PRAG1",
  "term_label": "Unknown cellular component"
}